{
  "gene_symbol": "YY1AP1",
  "term_label": "Unknown biological process",
  "term_id": "UNKNOWN:0002",
  "gene": "UniProtKB:Q9H869",
  "gene_name": "YY1-associated protein 1"
}